{
  "term_id": "GO:0007420",
  "gene": "UniProtKB:Q86WK7",
  "term_label": "brain development",
  "gene_name": "Amphoterin-induced protein 3",
  "gene_symbol": "AMIGO3"
}